vascular endothelial cell response to pulsatile fluid shear stress [GO:0097705] (biological process) Definition: Any response to pulsatile fluid shear stress that occurs in a vascular endothelial cell. References: PMID:21768538 Sources: GOC:BHF, GOC:BHF_miRNA, GOC:bc Also known as: blood vessel endothelial cell response to pulsatile fluid shear stress Relationships: is a type of vascular endothelial cell response to fluid shear stress [GO:0097699]; is a type of GO:0097703